{
  "gene_name": "Dynein axonemal heavy chain 11",
  "term_label": "cilium movement involved in cell motility",
  "term_id": "GO:0060294",
  "gene": "UniProtKB:Q96DT5",
  "gene_symbol": "DNAH11"
}